{
  "gene_symbol": "CC2D2B",
  "term_label": "Unknown molecular function",
  "term_id": "UNKNOWN:0001",
  "gene": "UniProtKB:Q6DHV5",
  "gene_name": "Protein CC2D2B"
}